{
  "term_id": "GO:0007288",
  "gene": "UniProtKB:Q9H892",
  "gene_symbol": "TTC12",
  "term_label": "sperm axoneme assembly",
  "gene_name": "Tetratricopeptide repeat protein 12"
}